{
  "term_label": "fibroblast growth factor receptor signaling pathway",
  "term_id": "GO:0008543",
  "gene_name": "Fibroblast growth factor receptor 4",
  "gene": "UniProtKB:P22455",
  "gene_symbol": "FGFR4"
}